{
  "gene_name": "Protein transport protein Sec31A",
  "term_label": "structural molecule activity",
  "gene": "UniProtKB:O94979",
  "term_id": "GO:0005198",
  "gene_symbol": "SEC31A"
}